{
  "gene_symbol": "OVOL1",
  "gene": "UniProtKB:O14753",
  "term_id": "GO:0000981",
  "gene_name": "Putative transcription factor Ovo-like 1",
  "term_label": "DNA-binding transcription factor activity, RNA polymerase II-specific"
}